{
  "term_id": "GO:0031444",
  "gene_name": "Troponin T, slow skeletal muscle",
  "term_label": "slow-twitch skeletal muscle fiber contraction",
  "gene_symbol": "TNNT1",
  "gene": "UniProtKB:P13805"
}